{
  "term_label": "14-3-3 protein binding",
  "gene": "UniProtKB:Q9NX09",
  "term_id": "GO:0071889",
  "gene_name": "DNA damage-inducible transcript 4 protein",
  "gene_symbol": "DDIT4"
}